{
  "gene_symbol": "DAZAP1",
  "gene": "UniProtKB:Q96EP5",
  "term_label": "perinuclear region of cytoplasm",
  "term_id": "GO:0048471",
  "gene_name": "DAZ-associated protein 1"
}